{
  "gene_symbol": "GORAB",
  "term_id": "UNKNOWN:0003",
  "term_label": "Unknown cellular component",
  "gene_name": "RAB6-interacting golgin",
  "gene": "UniProtKB:Q5T7V8"
}